{
  "gene_symbol": "TVP23A",
  "gene": "UniProtKB:A6NH52",
  "term_label": "vesicle-mediated transport",
  "gene_name": "Golgi apparatus membrane protein TVP23 homolog A",
  "term_id": "GO:0016192"
}